regulation of interleukin-11 production [GO:0032654] (biological process) Relationships: is a type of GO:0001817; regulates interleukin-11 production [GO:0032614] Also known as: regulation of IL-11 production, regulation of interleukin-11 biosynthetic process, regulation of interleukin-11 secretion References: PMID:29286137 Sources: GOC:mah Subtypes: negative regulation of interleukin-11 production [GO:0032694], positive regulation of interleukin-11 production [GO:0032734] Definition: Any process that modulates the frequency, rate, or extent of interleukin-11 production.